{
  "gene_name": "Immunoglobulin kappa variable 6D-21",
  "term_id": "UNKNOWN:0001",
  "term_label": "Unknown molecular function",
  "gene_symbol": "IGKV6D-21",
  "gene": "UniProtKB:A0A0A0MT36"
}